detection of temperature stimulus involved in thermoception [GO:0050960] (BP) Subtypes: detection of hot stimulus involved in thermoception [GO:0120168], detection of cold stimulus involved in thermoception [GO:0120169] Definition: The series of events in which a temperature stimulus is received and converted into a molecular signal as part of thermoception. Also known as: sensory detection of temperature stimulus during thermoception, sensory detection of thermal stimulus during thermoception, sensory transduction of temperature stimulus during thermoception, sensory transduction of thermal stimulus during thermoception, thermoception, sensory detection of temperature stimulus, thermoception, sensory detection of thermal stimulus, thermoception, sensory transduction of temperature stimulus, thermoception, sensory transduction of thermal stimulus Sources: GOC:ai, GOC:dos Relationships: is a type of detection of temperature stimulus involved in sensory perception [GO:0050961]; is part of thermoception [GO:0050955]